{
  "gene_symbol": "POLR1D",
  "term_id": "GO:0005736",
  "term_label": "RNA polymerase I complex",
  "gene_name": "DNA-directed RNA polymerases I and III subunit RPAC2",
  "gene": "UniProtKB:P0DPB6"
}